negative regulation of megakaryocyte differentiation [GO:0045653] (biological process) Relationships: is a type of GO:0045638; is a type of regulation of megakaryocyte differentiation [GO:0045652]; RO_0002212 megakaryocyte differentiation [GO:0030219] Also known as: down regulation of megakaryocyte differentiation, down-regulation of megakaryocyte differentiation, downregulation of megakaryocyte differentiation, inhibition of megakaryocyte differentiation Sources: GOC:go_curators Definition: Any process that stops, prevents, or reduces the frequency, rate or extent of megakaryocyte differentiation.